{
  "gene": "UniProtKB:O95428",
  "term_label": "Unknown cellular component",
  "gene_name": "Papilin",
  "gene_symbol": "PAPLN",
  "term_id": "UNKNOWN:0003"
}